{
  "term_id": "UNKNOWN:0003",
  "term_label": "Unknown cellular component",
  "gene_name": "Protein FAM218A",
  "gene_symbol": "FAM218A",
  "gene": "UniProtKB:Q96MZ4"
}